regulation of brown fat cell differentiation [GO:0090335] (biological process) Relationships: is a type of regulation of fat cell differentiation [GO:0045598]; regulates GO:0050873 Subtypes: positive regulation of brown fat cell differentiation [GO:0090336], GO:1903444 Sources: GOC:tb Definition: Any process that modulates the rate, frequency, or extent of brown fat cell differentiation. Brown fat cell differentiation is the process in which a relatively unspecialized cell acquires specialized features of a brown adipocyte, an animal connective tissue cell involved in adaptive thermogenesis. Brown adipocytes contain multiple small droplets of triglycerides and a high number of mitochondria.